{
  "gene_name": "Aminomethyltransferase, mitochondrial",
  "gene": "UniProtKB:P48728",
  "term_id": "GO:0004047",
  "term_label": "aminomethyltransferase activity",
  "gene_symbol": "AMT"
}